methane biosynthetic process from methylamine [GO:2001128] (biological process) Relationships: is a type of GO:0015948; is_a GO:0030416 Sources: GOC:mengo_curators Definition: The chemical reactions and pathways resulting in the formation of a methane from a methylamine. Regulation: regulated by regulation of methane biosynthetic process from methylamine [GO:1900348]; negatively regulated by GO:1900349; positively regulated by positive regulation of methane biosynthetic process from methylamine [GO:1900350]